{
  "gene": "UniProtKB:Q8TA94",
  "gene_symbol": "ZNF563",
  "gene_name": "Zinc finger protein 563",
  "term_id": "GO:0000977",
  "term_label": "RNA polymerase II transcription regulatory region sequence-specific DNA binding"
}